{
  "gene_symbol": "DEPDC5",
  "term_id": "GO:0010508",
  "term_label": "positive regulation of autophagy",
  "gene": "UniProtKB:O75140",
  "gene_name": "GATOR complex protein DEPDC5"
}